{
  "term_id": "UNKNOWN:0003",
  "gene_name": "Phosphotriesterase-related protein",
  "gene_symbol": "PTER",
  "gene": "UniProtKB:Q96BW5",
  "term_label": "Unknown cellular component"
}